D(-)-lactate biosynthetic process from pyruvate [GO:0019245] (biological process) Also known as: D(-)-lactate anabolism from pyruvate, D(-)-lactate formation from pyruvate, D(-)-lactate synthesis from pyruvate Relationships: is a type of lactate biosynthetic process from pyruvate [GO:0019244]; has part D-lactate dehydrogenase (NAD+) activity [GO:0008720] Sources: GOC:go_curators Definition: The chemical reactions and pathways resulting in the formation of D(-)-lactate from other compounds, including pyruvate.